mRNA trans splicing, via spliceosome [GO:0000365] (BP) Definition: The joining together of exons from two different primary transcripts of messenger RNA (mRNA) via a spliceosomal mechanism, so that mRNA consisting only of the joined exons is produced. Relationships: is a type of mRNA splicing, via spliceosome [GO:0000398] Also known as: nuclear mRNA trans splicing, via spliceosome, nuclear mRNA trans splicing, via U2-type spliceosome Subtypes: mRNA alternative trans-splicing [GO:0000366], mRNA trans splicing, SL addition [GO:0045291] References: PMID:18458335 Sources: GOC:krc, ISBN:0879695897